{
  "gene_name": "Estrogen-related receptor gamma",
  "gene": "UniProtKB:P62508",
  "gene_symbol": "ESRRG",
  "term_label": "nucleus",
  "term_id": "GO:0005634"
}